{
  "gene_name": "Transcription initiation factor TFIID subunit 9B",
  "gene_symbol": "TAF9B",
  "term_label": "RNA polymerase II general transcription initiation factor activity",
  "term_id": "GO:0016251",
  "gene": "UniProtKB:Q9HBM6"
}